{
  "term_label": "Unknown cellular component",
  "gene_symbol": "VAT1L",
  "gene": "UniProtKB:Q9HCJ6",
  "gene_name": "Synaptic vesicle membrane protein VAT-1 homolog-like",
  "term_id": "UNKNOWN:0003"
}